DNA double-strand break processing involved in repair via single-strand annealing [GO:0010792] (biological process) Relationships: is a type of DNA double-strand break processing [GO:0000729]; is part of double-strand break repair via single-strand annealing [GO:0045002] Definition: The 5' to 3' exonucleolytic resection of the DNA at the site of the break to form a 3' single-strand DNA overhang that results in the repair of a double strand break via single-strand annealing. Sources: GOC:dph, GOC:tb